{
  "term_id": "UNKNOWN:0002",
  "gene_symbol": "HEBP1",
  "gene": "UniProtKB:Q9NRV9",
  "term_label": "Unknown biological process",
  "gene_name": "Heme-binding protein 1"
}